{
  "term_id": "GO:0005737",
  "gene": "UniProtKB:Q969P5",
  "gene_name": "F-box only protein 32",
  "gene_symbol": "FBXO32",
  "term_label": "cytoplasm"
}